{
  "gene_name": "Uracil nucleotide_cysteinyl leukotriene receptor",
  "term_id": "GO:0004930",
  "gene": "UniProtKB:Q13304",
  "gene_symbol": "GPR17",
  "term_label": "G protein-coupled receptor activity"
}